{
  "gene": "UniProtKB:Q9NVF7",
  "term_label": "protein polyubiquitination",
  "term_id": "GO:0000209",
  "gene_name": "F-box only protein 28",
  "gene_symbol": "FBXO28"
}